{
  "gene_name": "G-protein coupled receptor 62",
  "term_label": "ligand-independent adenylate cyclase-activating G protein-coupled receptor signaling pathway",
  "term_id": "GO:0038035",
  "gene_symbol": "GPR62",
  "gene": "UniProtKB:Q9BZJ7"
}